{
  "term_label": "ubiquitin conjugating enzyme binding",
  "gene_symbol": "DCUN1D1",
  "gene_name": "DCN1-like protein 1",
  "gene": "UniProtKB:Q96GG9",
  "term_id": "GO:0031624"
}